{
  "term_label": "G protein-coupled serotonin receptor activity",
  "gene_symbol": "HTR1F",
  "gene_name": "5-hydroxytryptamine receptor 1F",
  "gene": "UniProtKB:P30939",
  "term_id": "GO:0004993"
}